{
  "gene_name": "Neuronal tyrosine-phosphorylated phosphoinositide-3-kinase adapter 1",
  "gene": "UniProtKB:Q6ZVC0",
  "term_id": "UNKNOWN:0003",
  "term_label": "Unknown cellular component",
  "gene_symbol": "NYAP1"
}